{
  "term_id": "GO:0004820",
  "term_label": "glycine-tRNA ligase activity",
  "gene": "UniProtKB:P41250",
  "gene_symbol": "GARS1",
  "gene_name": "Glycine--tRNA ligase"
}